{
  "term_label": "phosphatidylinositol-3-phosphate binding",
  "term_id": "GO:0032266",
  "gene_name": "Pleckstrin homology domain-containing family A member 4",
  "gene_symbol": "PLEKHA4",
  "gene": "UniProtKB:Q9H4M7"
}